wybutosine biosynthetic process [GO:0031591] (biological process) Note: Note that wybutosine is a hypermodified G-residue, formerly called the Y-base, and its derivatives are exclusively found at position 37 (anticodon loop) of tRNAPhe. Sources: GOC:hjd, GOC:mah, RNAmods:037 Relationships: is a type of tRNA modification [GO:0006400]; is a type of glycosyl compound biosynthetic process [GO:1901659] Also known as: yW biosynthesis, yW biosynthetic process Definition: The chemical reactions and pathways resulting in the formation of wybutosine, 3H-imidazo[1,2-alpha]purine-7-butanoic acid, 4,9-dihydro- alpha-[(methoxycarbonyl)amino]- 4,6-dimethyl-9-oxo- 3-beta-D-ribofuranosyl methyl ester, a modified nucleoside found in some tRNA molecules.